{
  "term_label": "Unknown biological process",
  "gene_symbol": "PGGT1B",
  "term_id": "UNKNOWN:0002",
  "gene_name": "Geranylgeranyl transferase type-1 subunit beta",
  "gene": "UniProtKB:P53609"
}